spindle microtubule [GO:0005876] (cellular component) Definition: Any microtubule that is part of a mitotic or meiotic spindle; anchored at one spindle pole. Sources: ISBN:0815316194 Relationships: is a type of GO:0005874; is part of spindle [GO:0005819] Subtypes: astral microtubule [GO:0000235], polar microtubule [GO:0005827], kinetochore microtubule [GO:0005828], GO:1990498